negative regulation of spindle checkpoint [GO:0090233] (biological process) Note: Note that this term should not be used for direct manual annotation as it should always be possible to specify the type of checkpoint (i.e mitotic spindle or DNA damage etc). Subtypes: negative regulation of mitotic spindle assembly checkpoint signaling [GO:0140499] Definition: Any process that decreases the rate, frequency, or extent of the spindle checkpoint, a cell cycle checkpoint that delays the metaphase/anaphase transition until the spindle is correctly assembled and oriented, and chromosomes are attached to the spindle. Relationships: is a type of regulation of spindle checkpoint [GO:0090231]; is a type of negative regulation of cell cycle checkpoint [GO:1901977]; negatively regulates GO:0031577 Sources: GOC:ascb_2009, GOC:dph, GOC:tb Also known as: spindle checkpoint silencing